{
  "gene_name": "Ly6_PLAUR domain-containing protein 1",
  "gene_symbol": "LYPD1",
  "gene": "UniProtKB:Q8N2G4",
  "term_label": "Unknown cellular component",
  "term_id": "UNKNOWN:0003"
}